habenula development [GO:0021986] (biological process) Relationships: is a type of anatomical structure development [GO:0048856]; is part of epithalamus development [GO:0021538] Sources: GOC:cls, GOC:dgh, GOC:dph, GOC:jid, GO_REF:0000021 Definition: The progression of the habenula over time from its initial formation until its mature state. The habenula is the group of nuclei that makes up the stalk of the pineal gland.